{
  "gene_symbol": "BNC2",
  "term_id": "UNKNOWN:0001",
  "term_label": "Unknown molecular function",
  "gene": "UniProtKB:Q6ZN30",
  "gene_name": "Zinc finger protein basonuclin-2"
}